negative regulation of viral translation [GO:1904972] (BP) Also known as: down regulation of viral protein anabolism, down regulation of viral protein biosynthesis, down regulation of viral protein biosynthetic process, down regulation of viral protein formation, down regulation of viral protein synthesis, down regulation of viral translation, down-regulation of viral protein anabolism, down-regulation of viral protein biosynthesis, down-regulation of viral protein biosynthetic process, down-regulation of viral protein formation, down-regulation of viral protein synthesis, down-regulation of viral translation, downregulation of viral protein anabolism, downregulation of viral protein biosynthesis, downregulation of viral protein biosynthetic process, downregulation of viral protein formation, downregulation of viral protein synthesis, downregulation of viral translation, negative regulation of viral protein anabolism, negative regulation of viral protein biosynthesis, negative regulation of viral protein biosynthetic process, negative regulation of viral protein formation, negative regulation of viral protein synthesis, inhibition of viral protein anabolism, inhibition of viral protein biosynthesis, inhibition of viral protein biosynthetic process, inhibition of viral protein formation, inhibition of viral protein synthesis, inhibition of viral translation Definition: Any process that stops, prevents or reduces the frequency, rate or extent of viral translation. Relationships: is a type of negative regulation of viral process [GO:0048525]; is a type of GO:1904971; negatively regulates GO:0019081 References: PMID:19666601 Sources: GOC:TermGenie, GOC:bhm, GO_REF:0000058